R1/R6 cell fate commitment [GO:0007462] (biological process) Definition: The process in which the R1/R6 photoreceptors commit to their cell fate. R1 and R6 are paired photoreceptors which contribute the outer rhabdomeres. Relationships: is a type of compound eye photoreceptor fate commitment [GO:0001752]; is part of GO:0048052 References: PMID:3076112, PMID:3937883